{
  "gene_symbol": "CFAP298",
  "gene_name": "Cilia- and flagella-associated protein 298",
  "gene": "UniProtKB:P57076",
  "term_label": "Unknown molecular function",
  "term_id": "UNKNOWN:0001"
}